{
  "gene_name": "Archaemetzincin-1",
  "term_id": "UNKNOWN:0003",
  "term_label": "Unknown cellular component",
  "gene": "UniProtKB:Q400G9",
  "gene_symbol": "AMZ1"
}